response to ketone [GO:1901654] (biological process) Subtypes: response to progesterone [GO:0032570], response to vitamin K [GO:0032571], response to testosterone [GO:0033574], response to hydroxyisoflavone [GO:0033594], GO:0034695, response to ecdysone [GO:0035075], response to iloperidone [GO:0036287], response to cycloheximide [GO:0046898], response to corticosterone [GO:0051412], response to cortisone [GO:0051413], GO:0051414, response to methylglyoxal [GO:0051595], response to dexamethasone [GO:0071548], response to prostaglandin D [GO:0071798], response to tetracycline [GO:1901326], response to rapamycin [GO:1901355], GO:1901557, cellular response to ketone [GO:1901655], response to ketamine [GO:1901986], response to docetaxel trihydrate [GO:1902519], response to doxorubicin [GO:1902520], response to 4'-epidoxorubicin [GO:1902522], response to plumbagin [GO:1902708], response to differentiation-inducing factor 1 [GO:1903013], response to dehydroepiandrosterone [GO:1903494], response to 11-deoxycorticosterone [GO:1903496], GO:1904044, response to forskolin [GO:1904321], response to nocodazole [GO:1904402], response to wortmannin [GO:1904567], response to phorbol 13-acetate 12-myristate [GO:1904627], response to curcumin [GO:1904643], GO:1904647, response to haloperidol [GO:1905119], GO:1905960 Definition: A response that results in a state of tolerance to ketone. Also known as: process resulting in tolerance to ketone Relationships: is_a response to oxygen-containing compound [GO:1901700] References: PMID:23356676 Sources: GOC:mengo_curators